{
  "term_id": "GO:0005829",
  "gene_name": "SEC14-like protein 1",
  "gene": "UniProtKB:Q92503",
  "gene_symbol": "SEC14L1",
  "term_label": "cytosol"
}